{
  "gene_name": "Putative 3-phosphoinositide-dependent protein kinase 2",
  "term_id": "UNKNOWN:0003",
  "gene_symbol": "PDPK2P",
  "gene": "UniProtKB:Q6A1A2",
  "term_label": "Unknown cellular component"
}